{
  "term_id": "GO:0005795",
  "term_label": "Golgi stack",
  "gene": "UniProtKB:O60763",
  "gene_name": "General vesicular transport factor p115",
  "gene_symbol": "USO1"
}